{
  "gene_symbol": "APOC3",
  "term_label": "triglyceride catabolic process",
  "gene_name": "Apolipoprotein C-III",
  "term_id": "GO:0019433",
  "gene": "UniProtKB:P02656"
}